peptidase inhibitor activity [GO:0030414] (molecular function) Subtypes: endopeptidase inhibitor activity [GO:0004866], peptidyl-dipeptidase inhibitor activity [GO:0060422] Definition: Binds to and stops, prevents or reduces the activity of a peptidase, any enzyme that catalyzes the hydrolysis peptide bonds. Relationships: is a type of enzyme inhibitor activity [GO:0004857]; is a type of peptidase regulator activity [GO:0061134]; negatively regulates GO:0008233 Also known as: protease inhibitor activity Sources: GOC:jl